{
  "gene_name": "Golgin subfamily A member 6D",
  "term_id": "GO:0000137",
  "term_label": "Golgi cis cisterna",
  "gene_symbol": "GOLGA6D",
  "gene": "UniProtKB:P0CG33"
}